{
  "term_id": "GO:0005829",
  "term_label": "cytosol",
  "gene_name": "Polyadenylate-binding protein 4",
  "gene_symbol": "PABPC4",
  "gene": "UniProtKB:Q13310"
}